geranylgeranyltransferase type III activity [GO:0170068] (molecular function) Relationships: is a type of GO:0004661 Definition: Catalyzes the covalent addition of a geranylgeranyl group to a mono-farnesylated substrate via a thioether linkage to a cysteine residue located within a conserved C-terminal tandem cysteine motif (CCAIM or CCIIM) that is used in substrate recognition. Known substrates include mono-farnesylated Golgi SNARE proteins. References: PMID:32128853, PMID:33035318, PMID:35628237, PMID:40049413 Also known as: GGTase-3 activity, GGTase-III activity, GGTase3 activity, Geranylgeranyl transferase type-3 activity, geranylgeranyltransferase type 3 activity